positive regulation of T cell apoptotic process [GO:0070234] (biological process) Definition: Any process that activates or increases the frequency, rate or extent of T cell death by apoptotic process. Sources: GOC:add, GOC:mtg_apoptosis, ISBN:0781765196 Also known as: positive regulation of T lymphocyte apoptosis, positive regulation of T-cell apoptosis, positive regulation of T-lymphocyte apoptosis, positive regulation of programmed cell death of T cells by apoptosis, up regulation of T cell apoptosis, up-regulation of T cell apoptosis, upregulation of T cell apoptosis, activation of T cell apoptosis, positive regulation of T cell apoptosis, stimulation of T cell apoptosis Relationships: is_a GO:0070230; is_a regulation of T cell apoptotic process [GO:0070232]; RO_0002213 T cell apoptotic process [GO:0070231] Subtypes: positive regulation of activation-induced cell death of T cells [GO:0070237], GO:0070241, positive regulation of thymocyte apoptotic process [GO:0070245], positive regulation of activated CD4-positive, alpha-beta T cell apoptotic process [GO:1905401], GO:1905404